regulation of translation involved in anterior/posterior axis specification [GO:0060815] (biological process) Sources: GOC:dph, GOC:sdb_2009, GOC:tb Definition: Any process that modulates the frequency, rate or extent of translation of mRNAs that contribute to the specification of the anterior/posterior axis. Relationships: is a type of regulation of translation [GO:0006417]; is part of anterior/posterior axis specification [GO:0009948]